sphingomyelin synthase activity [GO:0033188] (molecular function) Definition: Catalysis of the reaction: 1,2-diacyl-sn-glycero-3-phosphocholine + ceramide = 1,2-diacyl-sn-glycerol + sphingomyelin. Sources: EC:2.7.8.27, RHEA:18765 Also known as: SM synthase activity, SMS1, SMS2, ceramide:phosphatidylcholine cholinephosphotransferase activity, phosphatidylcholine:ceramide cholinephosphotransferase activity Relationships: is a type of phosphotransferase activity, for other substituted phosphate groups [GO:0016780]